{
  "gene": "UniProtKB:Q9H7D0",
  "term_label": "small GTPase binding",
  "gene_symbol": "DOCK5",
  "term_id": "GO:0031267",
  "gene_name": "Dedicator of cytokinesis protein 5"
}